{
  "term_label": "exocytosis",
  "term_id": "GO:0006887",
  "gene_symbol": "SYTL5",
  "gene": "UniProtKB:Q8TDW5",
  "gene_name": "Synaptotagmin-like protein 5"
}